{
  "gene_name": "Nitric oxide synthase 3",
  "term_id": "GO:0006809",
  "term_label": "nitric oxide biosynthetic process",
  "gene_symbol": "NOS3",
  "gene": "UniProtKB:P29474"
}